neuropore closure [GO:0021995] (biological process) Sources: GOC:cls, GOC:dgh, GOC:dph, GOC:jid, GO_REF:0000021 Relationships: is a type of morphogenesis of embryonic epithelium [GO:0016331]; is part of neural tube closure [GO:0001843] Definition: The process of joining together the neural folds at either end of the neural tube.